{
  "term_id": "UNKNOWN:0002",
  "term_label": "Unknown biological process",
  "gene": "UniProtKB:P57078",
  "gene_symbol": "RIPK4",
  "gene_name": "Receptor-interacting serine_threonine-protein kinase 4"
}